{
  "gene": "UniProtKB:Q9NR09",
  "gene_name": "Baculoviral IAP repeat-containing protein 6",
  "gene_symbol": "BIRC6",
  "term_id": "GO:0061631",
  "term_label": "ubiquitin conjugating enzyme activity"
}